{
  "term_id": "GO:0005634",
  "gene_symbol": "SHMT1",
  "term_label": "nucleus",
  "gene": "UniProtKB:P34896",
  "gene_name": "Serine hydroxymethyltransferase, cytosolic"
}